{
  "gene_name": "Protein N-terminal glutamine amidohydrolase",
  "term_id": "GO:0005634",
  "gene_symbol": "NTAQ1",
  "term_label": "nucleus",
  "gene": "UniProtKB:Q96HA8"
}